nucleotide diphosphokinase activity [GO:0050148] (molecular function) Sources: RHEA:12713 Relationships: is_a GO:0016778 Also known as: nucleotide pyrophosphokinase activity, ATP nucleotide 3'-pyrophosphokinase activity, ATP:nucleoside-5'-phosphate diphosphotransferase activity, ATP:nucleotide pyrophosphotransferase activity, nucleotide 3'-pyrophosphokinase activity Definition: Catalysis of the reaction: ATP + nucleoside 5'-phosphate = AMP + 5'-phosphonucleoside 3'-diphosphate.